{
  "term_label": "membrane organization",
  "term_id": "GO:0061024",
  "gene_symbol": "SAR1B",
  "gene_name": "GTP-binding protein SAR1b",
  "gene": "UniProtKB:Q9Y6B6"
}